malolactic enzyme activity [GO:0043883] (molecular function) References: PMID:3139053 Sources: RHEA:46276 Relationships: is a type of carboxy-lyase activity [GO:0016831] Note: This function is part of the process of degradation of L-malic acid by lactic acid bacteria. Also known as: MleS Definition: Catalysis of the reaction: (S)-malate + H+ = (S)-lactate + CO2.